Scrib-APC complex [GO:0034749] (cellular component) Also known as: hScrib-APC complex Note: Note that the gene/protein name 'APC' should not be confused with the abbreviation for 'anaphase promoting complex'. References: PMID:16611247 Definition: A protein complex that contains the Scribble protein (a cell polarity determinant) and the tumor suppressor protein adenomatous polyposis coli (APC); may be involved in the control of cell proliferation. Relationships: is a type of protein-containing complex [GO:0032991]; is part of GO:0005737